prostate glandular acinus development [GO:0060525] (biological process) References: PMID:18977204 Sources: GOC:dph Relationships: is a type of GO:0003006; is a type of anatomical structure development [GO:0048856]; is part of prostate gland development [GO:0030850] Definition: The progression of a glandular acinus of the prostate gland over time, from its initial formation to the mature structure. The glandular acini are the saclike structures of the gland.